{
  "term_label": "cilium assembly",
  "gene_symbol": "IFT52",
  "term_id": "GO:0060271",
  "gene_name": "Intraflagellar transport protein 52 homolog",
  "gene": "UniProtKB:Q9Y366"
}